beta-1,3-galactosyl-O-glycosyl-glycoprotein beta-1,3-N-acetylglucosaminyltransferase activity [GO:0047223] (molecular function) Relationships: is a type of acetylglucosaminyltransferase activity [GO:0008375]; is a type of catalytic activity, acting on a glycoprotein [GO:0140103] Sources: EC:2.4.1.146, MetaCyc:2.4.1.146-RXN Also known as: O-glycosyl-oligosaccharide-glycoprotein N-acetylglucosaminyltransferase II activity, UDP-N-acetyl-D-glucosamine:O-glycosyl-glycoprotein (N-acetyl-D-glucosamine to -D-galactose of beta-D-galactosyl-1,3-(N-acetyl-D-glucosaminyl-1,6)-N-acetyl-D-galactosaminyl-R) beta-1,3-N-acetyl-D-glucosaminyltransferase activity, elongation 3-beta-GalNAc-transferase activity, elongation 3beta-GalNAc-transferase activity, uridine diphosphoacetylglucosamine-mucin beta(1->3)-acetylglucosaminyltransferase (elongating) Definition: Catalysis of the reaction: beta-D-galactosyl-1,3-(N-acetyl-D-glucosaminyl-1,6)-N-acetyl-D-galactosaminyl-R + UDP-N-acetyl-D-glucosamine = N-acetyl-beta-D-glucosaminyl-1,3-beta-D-galactosyl-1,3-(N-acetyl-beta-D-glucosaminyl-1,6)-N-acetyl-D-galactosaminyl-R + UDP.